{
  "gene_name": "Cyclin-K",
  "term_id": "GO:0008024",
  "term_label": "cyclin/CDK positive transcription elongation factor complex",
  "gene_symbol": "CCNK",
  "gene": "UniProtKB:O75909"
}